positive regulation of arginine biosynthetic process [GO:1900080] (biological process) Relationships: is a type of GO:0062013; is a type of GO:1900079; is a type of GO:2000284; positively regulates L-arginine biosynthetic process [GO:0006526] Sources: GOC:TermGenie, GOC:dgf Definition: Any process that activates or increases the frequency, rate or extent of arginine biosynthetic process. Also known as: positive regulation of arginine anabolism, positive regulation of arginine biosynthesis, positive regulation of arginine formation, positive regulation of arginine synthesis, up regulation of arginine anabolism, up regulation of arginine biosynthesis, up regulation of arginine biosynthetic process, up regulation of arginine formation, up regulation of arginine synthesis, up-regulation of arginine anabolism, up-regulation of arginine biosynthesis, up-regulation of arginine biosynthetic process, up-regulation of arginine formation, up-regulation of arginine synthesis, upregulation of arginine anabolism, upregulation of arginine biosynthesis, upregulation of arginine biosynthetic process, upregulation of arginine formation, upregulation of arginine synthesis, activation of arginine anabolism, activation of arginine biosynthesis, activation of arginine biosynthetic process, activation of arginine formation, activation of arginine synthesis